{
  "term_id": "UNKNOWN:0003",
  "gene_name": "Ankyrin repeat domain-containing protein 10",
  "gene_symbol": "ANKRD10",
  "gene": "UniProtKB:Q9NXR5",
  "term_label": "Unknown cellular component"
}